positive regulation of t-circle formation [GO:1904431] (biological process) References: PMID:22579284 Sources: GOC:BHF, GOC:BHF_telomere, GOC:TermGenie, GOC:nc, GO_REF:0000058 Definition: Any process that activates or increases the frequency, rate or extent of t-circle formation. Relationships: is_a GO:0032206; is a type of GO:0044089; is a type of regulation of t-circle formation [GO:1904429]; positively regulates GO:0090656 Also known as: positive regulation of telomeric circle formation, up regulation of t-circle formation, up regulation of telomeric circle formation, up-regulation of t-circle formation, up-regulation of telomeric circle formation, upregulation of t-circle formation, upregulation of telomeric circle formation, activation of t-circle formation, activation of telomeric circle formation